{
  "term_label": "female gonad development",
  "gene_symbol": "CYP19A1",
  "term_id": "GO:0008585",
  "gene_name": "Aromatase",
  "gene": "UniProtKB:P11511"
}